methylgalactoside transport [GO:0015765] (biological process) Relationships: is a type of glycoside transport [GO:1901656] Sources: GOC:curators Definition: The directed movement of methylgalactoside into, out of or within a cell, or between cells, by means of some agent such as a transporter or pore. Methylgalactoside is a compound in which the H of the OH group on carbon-1 of galactose is replaced by a methyl group.